{
  "term_id": "GO:0030015",
  "gene_symbol": "CNOT8",
  "gene_name": "CCR4-NOT transcription complex subunit 8",
  "gene": "UniProtKB:Q9UFF9",
  "term_label": "CCR4-NOT core complex"
}